formyl-methanofuran dehydrogenase (tungsten enzyme) complex [GO:0044675] (cellular component) References: PMID:8125106, PMID:8575452 Sources: GOC:mengo_curators Relationships: is a type of catalytic complex [GO:1902494] Definition: A protein complex consisting of four polypeptides which also contains tungsten, a molybdopterin guanine dinucleotide, and iron-sulfur clusters. This protein complex catalyzes the reversible conversion of CO2 and methanofuran to formylmethanofuran during methanogenesis.